{
  "gene_name": "Voltage-dependent anion-selective channel protein 1",
  "term_id": "GO:0008308",
  "term_label": "voltage-gated monoatomic anion channel activity",
  "gene": "UniProtKB:P21796",
  "gene_symbol": "VDAC1"
}